insulin-like growth factor binding [GO:0005520] (molecular function) Definition: Binding to an insulin-like growth factor, any member of a group of polypeptides that are structurally homologous to insulin and share many of its biological activities, but are immunologically distinct from it. Sources: ISBN:0198506732 Also known as: IGF binding Relationships: is_a growth factor binding [GO:0019838] Subtypes: insulin-like growth factor I binding [GO:0031994], GO:0031995